response to benzene [GO:1901423] (biological process) Definition: Any process that results in a change in state or activity of a cell or an organism (in terms of movement, secretion, enzyme production, gene expression, etc.) as a result of a benzene stimulus. Sources: GOC:TermGenie, GOC:mengo_curators Relationships: is a type of response to chemical [GO:0042221] Regulation: regulated by regulation of response to benzene [GO:1901451]; negatively regulated by negative regulation of response to benzene [GO:1901452]; positively regulated by positive regulation of response to benzene [GO:1901453]